{
  "term_id": "GO:0042633",
  "gene": "UniProtKB:Q9BYQ9",
  "term_label": "hair cycle",
  "gene_name": "Keratin-associated protein 4-8",
  "gene_symbol": "KRTAP4-8"
}